{
  "term_label": "ubiquitin protein ligase binding",
  "term_id": "GO:0031625",
  "gene_name": "RING finger protein 37",
  "gene": "UniProtKB:O94941",
  "gene_symbol": "UBOX5"
}